positive regulation of fibroblast apoptotic process [GO:2000271] (biological process) Relationships: is a type of positive regulation of apoptotic process [GO:0043065]; is a type of regulation of fibroblast apoptotic process [GO:2000269]; positively regulates GO:0044346 Also known as: positive regulation of fibroblast apoptosis Definition: Any process that activates or increases the frequency, rate or extent of fibroblast apoptotic process. Sources: GOC:mtg_apoptosis, GOC:obol, GOC:yaf